{
  "term_label": "Unknown biological process",
  "gene": "UniProtKB:Q6ZS17",
  "term_id": "UNKNOWN:0002",
  "gene_name": "Rho family-interacting cell polarization regulator 1",
  "gene_symbol": "RIPOR1"
}